{
  "term_label": "cortical actin cytoskeleton",
  "gene_name": "Glia maturation factor beta",
  "gene": "UniProtKB:P60983",
  "gene_symbol": "GMFB",
  "term_id": "GO:0030864"
}